{
  "gene_symbol": "CARD6",
  "term_label": "Unknown cellular component",
  "term_id": "UNKNOWN:0003",
  "gene_name": "Caspase recruitment domain-containing protein 6",
  "gene": "UniProtKB:Q9BX69"
}